{
  "gene": "UniProtKB:P49682",
  "gene_symbol": "CXCR3",
  "term_id": "GO:0019957",
  "term_label": "C-C chemokine binding",
  "gene_name": "C-X-C chemokine receptor type 3"
}